sensory neuron axon guidance [GO:0097374] (biological process) Definition: The process in which the migration of an axon growth cone of a sensory neuron is directed to a specific target site in response to a combination of attractive and repulsive cues. A sensory neuron is an afferent neuron conveying sensory impulses. Sources: CL:0000101, GOC:pr Subtypes: spinal sensory neuron axon guidance [GO:0097375] Relationships: is a type of GO:0007411 Regulation: RO_0002211 by GO:1905489; negatively regulated by negative regulation of sensory neuron axon guidance [GO:1905490]; positively regulated by positive regulation of sensory neuron axon guidance [GO:1905491]